response to high light intensity [GO:0009644] (biological process) Definition: Any process that results in a change in state or activity of a cell or an organism (in terms of movement, secretion, enzyme production, gene expression, etc.) as a result of a high light intensity stimulus. Sources: GOC:go_curators Relationships: is a type of GO:0009642 Subtypes: photoinhibition [GO:0010205], response to high fluence blue light stimulus by blue high-fluence system [GO:0055121], cellular response to high light intensity [GO:0071486]